coreceptor activity [GO:0015026] (molecular function) Definition: Combining with an extracellular or intracellular messenger, and in cooperation with a nearby primary receptor, initiating a change in cell activity. Relationships: is a type of GO:0038023 Also known as: coreceptor, insoluble ligand activity, coreceptor, soluble ligand activity Sources: GOC:go_curators